DNA end binding [GO:0045027] (molecular function) Sources: GOC:jl Relationships: is a type of DNA binding [GO:0003677] Definition: Binding to DNA ends exposed by the creation of double-strand breaks (DSBs).